cellooligosaccharide metabolic process [GO:2000902] (biological process) Definition: The chemical reactions and pathways involving a cellooligosaccharide. Sources: GOC:mengo_curators Also known as: cellooligosaccharide metabolism Relationships: is a type of oligosaccharide metabolic process [GO:0009311] Subtypes: cellooligosaccharide catabolic process [GO:2000903]